{
  "term_id": "GO:0006357",
  "gene": "UniProtKB:Q12778",
  "gene_name": "Forkhead box protein O1",
  "gene_symbol": "FOXO1",
  "term_label": "regulation of transcription by RNA polymerase II"
}